{
  "gene": "UniProtKB:Q6PJG9",
  "term_label": "postsynaptic density membrane",
  "term_id": "GO:0098839",
  "gene_symbol": "LRFN4",
  "gene_name": "Leucine-rich repeat and fibronectin type-III domain-containing protein 4"
}